{
  "gene_name": "Spermatogenesis-associated protein 46",
  "term_id": "GO:0009566",
  "gene": "UniProtKB:Q5T0L3",
  "gene_symbol": "SPATA46",
  "term_label": "fertilization"
}